{
  "gene_symbol": "GAL",
  "gene": "UniProtKB:P22466",
  "term_label": "neuropeptide hormone activity",
  "term_id": "GO:0005184",
  "gene_name": "Galanin peptides"
}